virion nucleoid [GO:0039642] (cellular component) References: PMID:14291596 Sources: GOC:bm Definition: The region of a virion in which the nucleic acid is confined. Relationships: is a type of virion component [GO:0044423]